response to transition metal nanoparticle [GO:1990267] (biological process) Relationships: is a type of response to chemical [GO:0042221] Definition: Any process that results in a change in state or activity of a cell or an organism (in terms of movement, secretion, enzyme production, gene expression, etc.) as a result of a transition metal nanoparticle. References: PMID:23150627 Subtypes: response to gold nanoparticle [GO:1990268] Also known as: response to colloidal metal, response to neutral metal atoms